{
  "gene_name": "von Willebrand factor C domain-containing protein 2-like",
  "term_id": "GO:0030514",
  "gene_symbol": "VWC2L",
  "term_label": "negative regulation of BMP signaling pathway",
  "gene": "UniProtKB:B2RUY7"
}